{
  "term_id": "UNKNOWN:0001",
  "gene_symbol": "PLRG1",
  "term_label": "Unknown molecular function",
  "gene_name": "Pleiotropic regulator 1",
  "gene": "UniProtKB:O43660"
}